toxin export channel activity [GO:0000269] (MF) Sources: GOC:mtg_transport Relationships: is a type of GO:0015288; is a type of toxin transmembrane transporter activity [GO:0019534] Definition: Enables the energy independent passage of toxins, sized less than 1000 Da, across a membrane towards the outside of the cell. The transmembrane portions of porins consist exclusively of beta-strands which form a beta-barrel. They are found in the outer membranes of Gram-negative bacteria, mitochondria, plastids and possibly acid-fast Gram-positive bacteria.